{
  "gene": "UniProtKB:P51153",
  "term_label": "exocytosis",
  "term_id": "GO:0006887",
  "gene_name": "Ras-related protein Rab-13",
  "gene_symbol": "RAB13"
}